protein processing involved in protein targeting to mitochondrion [GO:0006627] (biological process) Definition: The cleavage of peptide bonds in proteins, usually near the N terminus, contributing to the process of import into the mitochondrion. Several different peptidases mediate cleavage of proteins destined for different mitochondrial compartments. References: PMID:12191769 Sources: GOC:mcc Also known as: mitochondrial processing, mitochondrial protein processing during import Relationships: is a type of mitochondrial protein processing [GO:0034982]; is part of protein targeting to mitochondrion [GO:0006626] Regulation: regulated by GO:1903216; negatively regulated by negative regulation of protein processing involved in protein targeting to mitochondrion [GO:1903217]